lytic vacuole membrane [GO:0098852] (cellular component) Definition: The lipid bilayer surrounding a lytic vacuole and separating its contents from the cytoplasm of the cell. Sources: GOC:dos Relationships: is a type of vacuolar membrane [GO:0005774]; BFO_0000050 GO:0000323 Subtypes: fungal-type vacuole membrane [GO:0000329], lysosomal membrane [GO:0005765]